sebaceous gland cell differentiation [GO:0001949] (biological process) References: PMID:15737203 Sources: GOC:mgi_curators Relationships: is a type of epidermal cell differentiation [GO:0009913]; is part of sebaceous gland development [GO:0048733] Subtypes: acinar cell of sebaceous gland differentiation [GO:1903680] Also known as: sebocytes differentiation Definition: The process in which a relatively unspecialized epidermal cell acquires the specialized features of a sebaceous gland cell.